{
  "gene_symbol": "COA4",
  "term_id": "UNKNOWN:0001",
  "term_label": "Unknown molecular function",
  "gene_name": "Cytochrome c oxidase assembly factor 4 homolog, mitochondrial",
  "gene": "UniProtKB:Q9NYJ1"
}